{
  "gene_symbol": "PLEKHA5",
  "gene": "UniProtKB:Q9HAU0",
  "term_label": "phosphatidylinositol-3,5-bisphosphate binding",
  "gene_name": "Pleckstrin homology domain-containing family A member 5",
  "term_id": "GO:0080025"
}